longitudinal axis specification [GO:0009942] (biological process) Relationships: is_a embryonic axis specification [GO:0000578]; is a type of GO:0003006; is part of GO:0009793 Definition: The establishment, maintenance and elaboration of the longitudinal axis. In plants, this is the axis that runs from the shoot to the root. Also known as: apical-basal pattern specification, longitudinal axis determination Sources: GOC:tb